nucleoside transmembrane transporter activity, down a concentration gradient [GO:0015395] (molecular function) Relationships: is a type of nucleoside transmembrane transporter activity [GO:0005337] Also known as: equilibrative nucleoside transporter activity, equilibrative nucleoside transmembrane transporter, nitrobenzyl-thioinosine-insensitive activity, equilibrative nucleoside transmembrane transporter, nitrobenzyl-thioinosine-sensitive activity Definition: Enables the transfer of a nucleoside, from one side of a membrane to the other, down the concentration gradient. References: PMID:10353709, PMID:11749958, PMID:12446811